{
  "gene": "UniProtKB:P16989",
  "term_id": "GO:0005634",
  "gene_name": "Y-box-binding protein 3",
  "gene_symbol": "YBX3",
  "term_label": "nucleus"
}